{
  "gene_name": "Bax inhibitor 1",
  "term_id": "GO:0060698",
  "gene": "UniProtKB:P55061",
  "term_label": "endoribonuclease inhibitor activity",
  "gene_symbol": "TMBIM6"
}